lacto-N-biosidase activity [GO:0047403] (molecular function) Sources: EC:3.2.1.140 Definition: Catalysis of the reaction: H2O + beta-D-Gal-(1,3)-beta-D-GlcNAc-(1,3)-beta-D-Gal-(1,4)-D-Glc = beta-D-Gal-(1,4)-D-Glc + beta-D-Gal-(1,3)-D-GlcNAc. Relationships: is a type of hydrolase activity, hydrolyzing O-glycosyl compounds [GO:0004553] Also known as: oligosaccharide lacto-N-biosylhydrolase activity